glutamate catabolic process to oxaloacetate [GO:0019554] (biological process) Definition: The chemical reactions and pathways resulting in the breakdown of glutamate into other compounds, including oxaloacetate. Relationships: is a type of oxaloacetate metabolic process [GO:0006107]; is a type of glutamate metabolic process [GO:0006536]; is a type of dicarboxylic acid catabolic process [GO:0043649]; is a type of dicarboxylic acid biosynthetic process [GO:0043650]; is a type of alpha-amino acid catabolic process [GO:1901606] Also known as: glutamate breakdown to oxaloacetate, glutamate degradation to oxaloacetate Sources: GOC:go_curators